{
  "term_label": "ubiquitin protein ligase activity",
  "gene_name": "E3 ubiquitin-protein ligase RNF144A",
  "gene": "UniProtKB:P50876",
  "term_id": "GO:0061630",
  "gene_symbol": "RNF144A"
}